{
  "term_label": "DNA-binding transcription factor activity, RNA polymerase II-specific",
  "gene_name": "Zinc finger protein 646",
  "gene": "UniProtKB:O15015",
  "gene_symbol": "ZNF646",
  "term_id": "GO:0000981"
}